{
  "term_label": "axon guidance",
  "gene_symbol": "ENAH",
  "term_id": "GO:0007411",
  "gene": "UniProtKB:Q8N8S7",
  "gene_name": "Protein enabled homolog"
}